collagen type IV trimer [GO:0005587] (cellular component) Relationships: is_a network-forming collagen trimer [GO:0098642]; is part of chicken-wire-like collagen network [GO:0140154] Definition: A collagen heterotrimer containing type IV alpha chains; [alpha1(IV)]2alpha2(IV) trimers are commonly observed, although more type IV alpha chains exist and may be present in type IV trimers; type IV collagen triple helices associate to form 3 dimensional nets within basement membranes. References: PMID:19693541, PMID:21421911